{
  "gene": "UniProtKB:Q6UXV1",
  "gene_name": "Izumo sperm-egg fusion protein 2",
  "gene_symbol": "IZUMO2",
  "term_label": "Unknown biological process",
  "term_id": "UNKNOWN:0002"
}